{
  "term_label": "Unknown cellular component",
  "gene": "UniProtKB:Q8TBF5",
  "term_id": "UNKNOWN:0003",
  "gene_symbol": "PIGX",
  "gene_name": "Phosphatidylinositol-glycan biosynthesis class X protein"
}